{
  "gene_name": "Serotransferrin",
  "term_label": "antibacterial humoral response",
  "term_id": "GO:0019731",
  "gene": "UniProtKB:P02787",
  "gene_symbol": "TF"
}